{
  "gene": "UniProtKB:Q9Y2G9",
  "term_id": "GO:0042393",
  "term_label": "histone binding",
  "gene_name": "Protein strawberry notch homolog 2",
  "gene_symbol": "SBNO2"
}